{
  "term_label": "intracellular signal transduction",
  "term_id": "GO:0035556",
  "gene_name": "Oxytocin-neurophysin 1",
  "gene": "UniProtKB:P01178",
  "gene_symbol": "OXT"
}